{
  "gene_name": "ADP-ribosylation factor-binding protein GGA1",
  "term_label": "small GTPase binding",
  "gene_symbol": "GGA1",
  "term_id": "GO:0031267",
  "gene": "UniProtKB:Q9UJY5"
}